{
  "gene": "UniProtKB:O15195",
  "term_id": "GO:0015629",
  "gene_name": "Villin-like protein",
  "gene_symbol": "VILL",
  "term_label": "actin cytoskeleton"
}